{
  "gene_symbol": "LOC105372440",
  "term_label": "Unknown molecular function",
  "gene": "UniProtKB:A0A1B0GTG8",
  "term_id": "UNKNOWN:0001",
  "gene_name": "Uncharacterized protein"
}